{
  "gene": "UniProtKB:Q6NT16",
  "gene_symbol": "SLC18B1",
  "term_id": "UNKNOWN:0002",
  "gene_name": "MFS-type transporter SLC18B1",
  "term_label": "Unknown biological process"
}